L-amino-acid dehydrogenase activity [GO:0050018] (molecular function) Definition: Catalysis of the reaction: an L-amino acid + H2O + NAD+ = a 2-oxo acid + NH3 + NADH. Sources: EC:1.4.1.5 Relationships: is a type of oxidoreductase activity, acting on the CH-NH2 group of donors, NAD or NADP as acceptor [GO:0016639] Also known as: L-amino-acid:NAD+ oxidoreductase (deaminating)